{
  "term_label": "termination of mitochondrial transcription",
  "gene_name": "Transcription termination factor 2, mitochondrial",
  "gene_symbol": "MTERF2",
  "gene": "UniProtKB:Q49AM1",
  "term_id": "GO:0006393"
}